{
  "gene_name": "Protein Jade-1",
  "gene_symbol": "JADE1",
  "term_label": "nucleus",
  "term_id": "GO:0005634",
  "gene": "UniProtKB:Q6IE81"
}